positive regulation of phosphatidylglycerol biosynthetic process [GO:1901353] (BP) Definition: Any process that activates or increases the frequency, rate or extent of phosphatidylglycerol biosynthetic process. References: PMID:12869188 Sources: GOC:TermGenie, GOC:dgf Also known as: positive regulation of phosphatidylglycerol anabolism, positive regulation of phosphatidylglycerol biosynthesis, positive regulation of phosphatidylglycerol formation, positive regulation of phosphatidylglycerol synthesis, up regulation of phosphatidylglycerol anabolism, up regulation of phosphatidylglycerol biosynthesis, up regulation of phosphatidylglycerol biosynthetic process, up regulation of phosphatidylglycerol formation, up regulation of phosphatidylglycerol synthesis, up-regulation of phosphatidylglycerol anabolism, up-regulation of phosphatidylglycerol biosynthesis, up-regulation of phosphatidylglycerol biosynthetic process, up-regulation of phosphatidylglycerol formation, up-regulation of phosphatidylglycerol synthesis, upregulation of phosphatidylglycerol anabolism, upregulation of phosphatidylglycerol biosynthesis, upregulation of phosphatidylglycerol biosynthetic process, upregulation of phosphatidylglycerol formation, upregulation of phosphatidylglycerol synthesis, activation of phosphatidylglycerol anabolism, activation of phosphatidylglycerol biosynthesis, activation of phosphatidylglycerol biosynthetic process, activation of phosphatidylglycerol formation, activation of phosphatidylglycerol synthesis Relationships: is a type of positive regulation of phospholipid biosynthetic process [GO:0071073]; is a type of GO:1901351; positively regulates phosphatidylglycerol biosynthetic process [GO:0006655]